{
  "gene_name": "5'(3')-deoxyribonucleotidase, mitochondrial",
  "term_id": "UNKNOWN:0003",
  "gene_symbol": "NT5M",
  "gene": "UniProtKB:Q9NPB1",
  "term_label": "Unknown cellular component"
}